{
  "term_label": "nucleoplasm",
  "term_id": "GO:0005654",
  "gene": "UniProtKB:Q6UXU6",
  "gene_symbol": "TMEM92",
  "gene_name": "Transmembrane protein 92"
}